{
  "gene_name": "Reelin domain-containing protein 1",
  "gene": "UniProtKB:A0A1B0GV85",
  "term_id": "GO:0016020",
  "term_label": "membrane",
  "gene_symbol": "REELD1"
}